{
  "gene_symbol": "GSC2",
  "gene": "UniProtKB:O15499",
  "gene_name": "Homeobox protein goosecoid-2",
  "term_id": "GO:0005634",
  "term_label": "nucleus"
}